{
  "gene_name": "Natural killer cells antigen CD94",
  "term_label": "positive regulation of natural killer cell mediated cytotoxicity",
  "gene_symbol": "KLRD1",
  "gene": "UniProtKB:Q13241",
  "term_id": "GO:0045954"
}